{
  "gene": "UniProtKB:Q96LA9",
  "gene_name": "Mas-related G-protein coupled receptor member X4",
  "term_id": "GO:0004930",
  "gene_symbol": "MRGPRX4",
  "term_label": "G protein-coupled receptor activity"
}